{
  "gene_symbol": "IGF1",
  "term_label": "insulin-like growth factor receptor signaling pathway",
  "gene": "UniProtKB:P05019",
  "gene_name": "Insulin-like growth factor I",
  "term_id": "GO:0048009"
}